negative regulation of inflammatory response to wounding [GO:0106015] (biological process) Definition: Any process that stops, prevents, or reduces the frequency, rate or extent of the inflammatory response to wounding. References: PMID:26022821 Sources: GOC:BHF, GOC:BHF_miRNA, GOC:rph Relationships: is a type of negative regulation of inflammatory response [GO:0050728]; is a type of GO:0106014; is a type of negative regulation of response to wounding [GO:1903035]; negatively regulates GO:0090594